negative regulation of vesicle fusion [GO:0031339] (biological process) Also known as: down regulation of vesicle fusion, down-regulation of vesicle fusion, downregulation of vesicle fusion, inhibition of vesicle fusion Definition: Any process that stops, prevents, or reduces the frequency, rate or extent of vesicle fusion. Sources: GOC:mah Relationships: is a type of negative regulation of organelle organization [GO:0010639]; is a type of regulation of vesicle fusion [GO:0031338]; is a type of negative regulation of transport [GO:0051051]; negatively regulates vesicle fusion [GO:0006906] Subtypes: negative regulation of synaptic vesicle fusion to presynaptic active zone membrane [GO:0031631], negative regulation of SNARE complex assembly [GO:0035544], GO:0048216, negative regulation of vesicle fusion with Golgi apparatus [GO:0106215], negative regulation of endosomal vesicle fusion [GO:1905362]